keratinocyte migration [GO:0051546] (biological process) Relationships: is a type of epithelial cell migration [GO:0010631] Regulation: regulated by regulation of keratinocyte migration [GO:0051547]; negatively regulated by negative regulation of keratinocyte migration [GO:0051548]; positively regulated by positive regulation of keratinocyte migration [GO:0051549] Sources: ISBN:0721662544 Definition: The directed movement of a keratinocyte, epidermal cells which synthesize keratin, from one site to another.